{
  "term_label": "protein tyrosine phosphatase activity",
  "gene_symbol": "PTPRD",
  "gene_name": "Receptor-type tyrosine-protein phosphatase delta",
  "term_id": "GO:0004725",
  "gene": "UniProtKB:P23468"
}